{
  "term_id": "GO:0005789",
  "gene": "UniProtKB:A1L3X0",
  "gene_symbol": "ELOVL7",
  "gene_name": "Elongation of very long chain fatty acids protein 7",
  "term_label": "endoplasmic reticulum membrane"
}